{
  "term_label": "plasma membrane",
  "gene_name": "SH3 domain-binding protein 1",
  "term_id": "GO:0005886",
  "gene": "UniProtKB:Q9Y3L3",
  "gene_symbol": "SH3BP1"
}